{
  "gene": "UniProtKB:O15037",
  "gene_symbol": "KHNYN",
  "term_label": "3'-UTR-mediated mRNA destabilization",
  "term_id": "GO:0061158",
  "gene_name": "Protein KHNYN"
}